{
  "gene_symbol": "MTSS1",
  "term_id": "GO:0015629",
  "term_label": "actin cytoskeleton",
  "gene_name": "Protein MTSS 1",
  "gene": "UniProtKB:O43312"
}